{
  "term_id": "GO:0006909",
  "gene_name": "Chemokine-like protein TAFA-4",
  "gene_symbol": "TAFA4",
  "term_label": "phagocytosis",
  "gene": "UniProtKB:Q96LR4"
}